{
  "gene_symbol": "UNC119",
  "gene": "UniProtKB:Q13432",
  "term_id": "GO:1900186",
  "term_label": "negative regulation of clathrin-dependent endocytosis",
  "gene_name": "Protein unc-119 homolog A"
}